{
  "gene_symbol": "POTEM",
  "term_label": "Unknown biological process",
  "term_id": "UNKNOWN:0002",
  "gene_name": "Putative POTE ankyrin domain family member M",
  "gene": "UniProtKB:A6NI47"
}